{
  "term_id": "GO:0006886",
  "gene_name": "ADP-ribosylation factor-like protein 5B",
  "gene_symbol": "ARL5B",
  "gene": "UniProtKB:Q96KC2",
  "term_label": "intracellular protein transport"
}